{
  "term_label": "sperm flagellum",
  "term_id": "GO:0036126",
  "gene": "UniProtKB:Q96M29",
  "gene_symbol": "TEKT5",
  "gene_name": "Tektin-5"
}